{
  "term_id": "GO:0005737",
  "gene_name": "GAS2-like protein 1",
  "gene_symbol": "GAS2L1",
  "term_label": "cytoplasm",
  "gene": "UniProtKB:Q99501"
}